{
  "term_label": "positive regulation of transcription by RNA polymerase II",
  "gene_name": "Myocyte-specific enhancer factor 2B",
  "gene": "UniProtKB:Q02080",
  "gene_symbol": "MEF2B",
  "term_id": "GO:0045944"
}